{
  "term_id": "GO:0006357",
  "gene": "UniProtKB:P41162",
  "term_label": "regulation of transcription by RNA polymerase II",
  "gene_name": "ETS translocation variant 3",
  "gene_symbol": "ETV3"
}